{
  "gene_name": "Superkiller complex protein 8",
  "term_id": "GO:0016593",
  "gene": "UniProtKB:Q9GZS3",
  "gene_symbol": "SKIC8",
  "term_label": "Cdc73/Paf1 complex"
}